positive regulation of collagen fibril organization [GO:1904028] (biological process) Also known as: positive regulation of collagen fibril organisation, positive regulation of fibrillar collagen organization, up regulation of collagen fibril organisation, up regulation of collagen fibril organization, up regulation of fibrillar collagen organization, up-regulation of collagen fibril organisation, up-regulation of collagen fibril organization, up-regulation of fibrillar collagen organization, upregulation of collagen fibril organisation, upregulation of collagen fibril organization, upregulation of fibrillar collagen organization, activation of collagen fibril organisation, activation of collagen fibril organization, activation of fibrillar collagen organization Definition: Any process that activates or increases the frequency, rate or extent of collagen fibril organization. References: PMID:25451920 Sources: GOC:TermGenie, GO_REF:0000058 Relationships: is a type of GO:1903055; is_a regulation of collagen fibril organization [GO:1904026]; positively regulates collagen fibril organization [GO:0030199]